positive regulation of mitotic cell cycle phase transition [GO:1901992] (biological process) References: PMID:22841721 Sources: GOC:TermGenie, GOC:mtg_cell_cycle Also known as: up regulation of mitotic cell cycle phase transition, up-regulation of mitotic cell cycle phase transition, upregulation of mitotic cell cycle phase transition, activation of mitotic cell cycle phase transition Subtypes: positive regulation of G2/M transition of mitotic cell cycle [GO:0010971], GO:0031536, GO:0045842, GO:1900087 Relationships: is a type of positive regulation of mitotic cell cycle [GO:0045931]; is a type of positive regulation of cell cycle phase transition [GO:1901989]; is a type of regulation of mitotic cell cycle phase transition [GO:1901990]; positively regulates mitotic cell cycle phase transition [GO:0044772] Definition: Any process that activates or increases the frequency, rate or extent of mitotic cell cycle phase transition.